L-phenylalanine biosynthetic process from chorismate via phenylpyruvate [GO:0033585] (biological process) Sources: GOC:go_curators Relationships: is a type of L-phenylalanine biosynthetic process [GO:0009094]; is a type of GO:0046417 Definition: The chemical reactions and pathways resulting in the formation of L-phenylalanine from other compounds, including chorismate, via the intermediate phenylpyruvate. Also known as: L-phenylalanine anabolism from chorismate via phenylpyruvate, L-phenylalanine biosynthesis from chorismate via phenylpyruvate, L-phenylalanine formation from chorismate via phenylpyruvate, L-phenylalanine synthesis from chorismate via phenylpyruvate